{
  "gene_name": "Tetratricopeptide repeat protein 4",
  "gene": "UniProtKB:O95801",
  "term_id": "GO:0006457",
  "term_label": "protein folding",
  "gene_symbol": "TTC4"
}